{
  "term_id": "GO:0023019",
  "term_label": "signal transduction involved in regulation of gene expression",
  "gene": "UniProtKB:O95813",
  "gene_name": "Cerberus",
  "gene_symbol": "CER1"
}